{
  "term_id": "GO:0050291",
  "term_label": "sphingosine N-acyltransferase activity",
  "gene_name": "Ceramide synthase 2",
  "gene_symbol": "CERS2",
  "gene": "UniProtKB:Q96G23"
}